leukocyte adhesive activation [GO:0050902] (BP) References: PMID:14680625, PMID:14708592, PMID:7507411, PMID:8600538 Sources: ISBN:0781735149 Also known as: leukocyte adhesive triggering Definition: The activation of loosely bound or rolling leukocytes by signals displayed on blood vessel endothelial cells, which is typically the second step in cellular extravasation. Relationships: is a type of GO:0045321; is part of cellular extravasation [GO:0045123]